{
  "gene_symbol": "ST20-AS1",
  "gene": "UniProtKB:Q8NBB2",
  "term_id": "UNKNOWN:0003",
  "gene_name": "Putative uncharacterized protein ST20-AS1",
  "term_label": "Unknown cellular component"
}